{
  "term_id": "GO:0030150",
  "gene_name": "Mitochondrial import receptor subunit TOM40 homolog",
  "gene_symbol": "TOMM40",
  "term_label": "protein import into mitochondrial matrix",
  "gene": "UniProtKB:O96008"
}